{
  "gene_symbol": "AGFG2",
  "gene": "UniProtKB:O95081",
  "gene_name": "Arf-GAP domain and FG repeat-containing protein 2",
  "term_label": "Unknown molecular function",
  "term_id": "UNKNOWN:0001"
}